{
  "term_id": "GO:0047617",
  "term_label": "fatty acyl-CoA hydrolase activity",
  "gene_symbol": "ACOT13",
  "gene_name": "Acyl-coenzyme A thioesterase 13",
  "gene": "UniProtKB:Q9NPJ3"
}